{
  "gene": "UniProtKB:O14795",
  "gene_name": "Protein unc-13 homolog B",
  "gene_symbol": "UNC13B",
  "term_id": "GO:0016082",
  "term_label": "synaptic vesicle priming"
}